nucleotide binding [GO:0000166] (MF) Definition: Binding to a nucleotide, any compound consisting of a nucleoside that is esterified with (ortho)phosphate or an oligophosphate at any hydroxyl group on the ribose or deoxyribose. Relationships: is a type of nucleoside phosphate binding [GO:1901265]; is a type of heterocyclic compound binding [GO:1901363] Sources: GOC:mah, ISBN:0198547684 Subtypes: methyl-CpG binding [GO:0008327], methyl-CpNpG binding [GO:0010428], GO:0010429, GO:0017076, pyrimidine nucleotide binding [GO:0019103], cyclic nucleotide binding [GO:0030551], deoxyribonucleotide binding [GO:0032552], GO:0032553, flavin adenine dinucleotide binding [GO:0050660]